regulation of respiratory gaseous exchange by nervous system process [GO:0002087] (biological process) Definition: A process carried out by the nervous system that is required for the proper control of respiratory gaseous exchange. This process occurs in the respiratory center of the brain in vertebrates. Also known as: neurological control of breathing, regulation of respiratory gaseous exchange by neurological system process References: PMID:12458206 Sources: GOC:dph, GOC:tb Relationships: is a type of regulation of respiratory system process [GO:0044065]; is a type of nervous system process [GO:0050877]